{
  "gene": "UniProtKB:Q8IYA6",
  "gene_name": "Cytoskeleton-associated protein 2-like",
  "gene_symbol": "CKAP2L",
  "term_label": "cytosol",
  "term_id": "GO:0005829"
}